alkylacetylglycerophosphatase activity [GO:0047647] (molecular function) Relationships: is a type of phosphatase activity [GO:0016791] Sources: RHEA:18221 Also known as: 1-alkyl-2-acetyl-sn-glycero-3-phosphate phosphohydrolase activity, 1-alkyl-2-lyso-sn-glycero-3-P:acetyl-CoA acetyltransferase activity, alkylacetylglycerophosphate phosphatase activity Definition: Catalysis of the reaction: 1-alkyl-2-acetyl-sn-glycerol 3-phosphate + H2O = 2-acetyl-1-alkyl-sn-glycerol + phosphate.